L-isoleucine biosynthetic process [GO:1901705] (biological process) Relationships: is a type of aspartate family amino acid biosynthetic process [GO:0009067]; is a type of isoleucine biosynthetic process [GO:0009097] Also known as: L-isoleucine anabolism, L-isoleucine biosynthesis, L-isoleucine formation, L-isoleucine synthesis Definition: The chemical reactions and pathways resulting in the formation of L-isoleucine. Sources: GOC:TermGenie